{
  "gene": "UniProtKB:Q6IQ26",
  "term_id": "GO:0005085",
  "gene_name": "DENN domain-containing protein 5A",
  "term_label": "guanyl-nucleotide exchange factor activity",
  "gene_symbol": "DENND5A"
}